seed morphogenesis [GO:0048317] (BP) Definition: The process in which the anatomical structures of the seed are generated and organized. Sources: GOC:go_curators Relationships: is a type of GO:0003006; is a type of post-embryonic plant morphogenesis [GO:0090698]; is part of seed development [GO:0048316]